{
  "gene_name": "Myelin proteolipid protein",
  "gene_symbol": "PLP1",
  "gene": "UniProtKB:P60201",
  "term_id": "GO:0022010",
  "term_label": "central nervous system myelination"
}